{
  "term_label": "phosphatidylethanolamine binding",
  "term_id": "GO:0008429",
  "gene_name": "Microtubule-associated proteins 1A_1B light chain 3B",
  "gene_symbol": "MAP1LC3B",
  "gene": "UniProtKB:Q9GZQ8"
}